{
  "term_label": "histone binding",
  "term_id": "GO:0042393",
  "gene_symbol": "L3MBTL2",
  "gene_name": "Lethal(3)malignant brain tumor-like protein 2",
  "gene": "UniProtKB:Q969R5"
}